{
  "term_id": "GO:0005925",
  "gene_symbol": "EVL",
  "gene": "UniProtKB:Q9UI08",
  "gene_name": "Ena_VASP-like protein",
  "term_label": "focal adhesion"
}